{
  "term_id": "GO:0005912",
  "term_label": "adherens junction",
  "gene": "UniProtKB:Q96RW7",
  "gene_symbol": "HMCN1",
  "gene_name": "Hemicentin-1"
}